kainate selective glutamate receptor signaling pathway [GO:0098991] (biological process) Sources: GOC:signaling, ISBN:9780071120005 Regulation: regulated by regulation of kainate selective glutamate receptor signaling pathway [GO:0106426] Relationships: is a type of ionotropic glutamate receptor signaling pathway [GO:0035235]; has part kainate selective glutamate receptor activity [GO:0015277] Definition: The series of molecular signals initiated by glutamate binding to an kainate-selective glutamate receptor on the surface of the target cell, followed by the movement of ions through a channel in the receptor complex, ending with the regulation of a downstream cellular process, e.g. transcription.